{
  "gene_name": "Lysosome-associated membrane glycoprotein 2",
  "term_label": "plasma membrane",
  "gene": "UniProtKB:P13473",
  "gene_symbol": "LAMP2",
  "term_id": "GO:0005886"
}